{
  "term_id": "GO:0003924",
  "gene_name": "Ras-related protein Rab-18",
  "gene": "UniProtKB:Q9NP72",
  "gene_symbol": "RAB18",
  "term_label": "GTPase activity"
}